regulation of Golgi to plasma membrane protein transport [GO:0042996] (biological process) Subtypes: negative regulation of Golgi to plasma membrane protein transport [GO:0042997], GO:0042998 Sources: GOC:jl Relationships: is a type of regulation of protein transport [GO:0051223]; is a type of regulation of vesicle-mediated transport [GO:0060627]; is a type of regulation of protein localization to plasma membrane [GO:1903076]; regulates GO:0043001 Definition: Any process that modulates the frequency, rate or extent of the transport of proteins from the Golgi to the plasma membrane.